{
  "gene": "UniProtKB:Q9H478",
  "gene_symbol": "KCNQ1DN",
  "term_id": "UNKNOWN:0003",
  "term_label": "Unknown cellular component",
  "gene_name": "KCNQ1 downstream neighbor protein"
}